RNA-protein covalent cross-linking [GO:0018144] (biological process) Subtypes: GO:0018259 Definition: The formation of a covalent cross-link between RNA and a protein. Relationships: is a type of GO:0018143 Sources: GOC:ma